{
  "gene_name": "Mitogen-activated protein kinase 1",
  "term_id": "GO:0005634",
  "gene_symbol": "MAPK1",
  "gene": "UniProtKB:P28482",
  "term_label": "nucleus"
}